medial fin development [GO:0033338] (biological process) Definition: The process whose specific outcome is the progression of a medial fin over time, from its formation to the mature structure. Sources: GOC:dgh Also known as: median fin development Relationships: is_a fin development [GO:0033333] Subtypes: anal fin development [GO:0033335], caudal fin development [GO:0033336], dorsal fin development [GO:0033337]